regulation of microglia differentiation [GO:0014006] (BP) Definition: Any process that modulates the frequency, rate or extent of microglia differentiation, the process in which a relatively unspecialized cell acquires specialized features of a microglial cell. Relationships: is a type of regulation of macrophage differentiation [GO:0045649]; is a type of regulation of glial cell differentiation [GO:0045685]; regulates microglia differentiation [GO:0014004] Sources: GOC:ef Subtypes: negative regulation of microglia differentiation [GO:0014007], positive regulation of microglia differentiation [GO:0014008] Also known as: regulation of microglial cell differentiation